{
  "gene_symbol": "THEM5",
  "gene_name": "Acyl-coenzyme A thioesterase THEM5",
  "gene": "UniProtKB:Q8N1Q8",
  "term_id": "GO:0035336",
  "term_label": "long-chain fatty-acyl-CoA metabolic process"
}